negative regulation of glycine import across plasma membrane [GO:1900924] (biological process) Sources: GOC:TermGenie Also known as: negative regulation of glycine import, down regulation of glycine import, down-regulation of glycine import, downregulation of glycine import, inhibition of glycine import Relationships: is a type of negative regulation of organic acid transport [GO:0032891]; is a type of negative regulation of transmembrane transport [GO:0034763]; is a type of negative regulation of amino acid transport [GO:0051956]; is a type of regulation of glycine import across plasma membrane [GO:1900923]; RO_0002212 glycine import across plasma membrane [GO:1903804] Definition: Any process that stops, prevents or reduces the frequency, rate or extent of glycine import into a cell.